{
  "gene": "UniProtKB:Q14721",
  "gene_symbol": "KCNB1",
  "term_label": "potassium channel regulator activity",
  "gene_name": "Potassium voltage-gated channel subfamily B member 1",
  "term_id": "GO:0015459"
}